inositol-1,3,4,5,6-pentakisphosphate kinase activity [GO:0000827] (molecular function) Definition: Catalysis of the reaction: ATP + 1D-myo-inositol 1,3,4,5,6-pentakisphosphate = ADP + diphospho-1D-myo-inositol tetrakisphosphate. The isomeric configuration of diphospho-1D-myo-inositol tetrakisphosphate is unknown. References: PMID:11311242 Sources: GOC:elh Relationships: is a type of GO:0016776; is a type of inositol phosphate kinase activity [GO:0180030]